{
  "gene": "UniProtKB:O95436",
  "gene_name": "Sodium-dependent phosphate transport protein 2B",
  "gene_symbol": "SLC34A2",
  "term_id": "GO:0030643",
  "term_label": "intracellular phosphate ion homeostasis"
}